{
  "gene": "UniProtKB:P24522",
  "gene_symbol": "GADD45A",
  "gene_name": "Growth arrest and DNA damage-inducible protein GADD45 alpha",
  "term_id": "UNKNOWN:0001",
  "term_label": "Unknown molecular function"
}